{
  "gene": "UniProtKB:Q8N6C8",
  "term_id": "GO:0005886",
  "gene_name": "Leukocyte immunoglobulin-like receptor subfamily A member 3",
  "term_label": "plasma membrane",
  "gene_symbol": "LILRA3"
}